{
  "gene_symbol": "AGTPBP1",
  "gene": "UniProtKB:Q9UPW5",
  "gene_name": "Cytosolic carboxypeptidase 1",
  "term_label": "tubulin binding",
  "term_id": "GO:0015631"
}